{
  "gene_symbol": "DAPL1",
  "term_label": "negative regulation of autophagy",
  "gene": "UniProtKB:A0PJW8",
  "gene_name": "Death-associated protein-like 1",
  "term_id": "GO:0010507"
}